{
  "gene": "UniProtKB:Q02083",
  "term_id": "UNKNOWN:0002",
  "term_label": "Unknown biological process",
  "gene_symbol": "NAAA",
  "gene_name": "N-acylethanolamine-hydrolyzing acid amidase"
}